{
  "term_label": "type I interferon-mediated signaling pathway",
  "gene_symbol": "C9JQL5",
  "gene": "UniProtKB:C9JQL5",
  "gene_name": "Putative dispanin subfamily A member 2d",
  "term_id": "GO:0060337"
}